{
  "term_label": "ubiquitin ligase complex scaffold activity",
  "gene": "UniProtKB:Q13618",
  "gene_name": "Cullin-3",
  "term_id": "GO:0160072",
  "gene_symbol": "CUL3"
}